{
  "term_label": "Unknown biological process",
  "gene_name": "MKI67 FHA domain-interacting nucleolar phosphoprotein",
  "term_id": "UNKNOWN:0002",
  "gene_symbol": "NIFK",
  "gene": "UniProtKB:Q9BYG3"
}